{
  "term_id": "UNKNOWN:0001",
  "gene": "UniProtKB:C9JQL5",
  "term_label": "Unknown molecular function",
  "gene_name": "Putative dispanin subfamily A member 2d",
  "gene_symbol": "C9JQL5"
}